{
  "term_id": "GO:0000978",
  "gene_name": "Replication initiator 1",
  "gene": "UniProtKB:Q9BWE0",
  "gene_symbol": "REPIN1",
  "term_label": "RNA polymerase II cis-regulatory region sequence-specific DNA binding"
}